{
  "term_label": "Unknown cellular component",
  "gene_symbol": "TMEM61",
  "gene": "UniProtKB:Q8N0U2",
  "term_id": "UNKNOWN:0003",
  "gene_name": "Transmembrane protein 61"
}